mating projection [GO:0005937] (CC) Sources: GOC:mcc Definition: The projection formed by unicellular fungi in response to mating pheromone. Relationships: is a type of plasma membrane bounded cell projection [GO:0120025] Also known as: conjugation tube, shmoo